{
  "term_label": "regulation of transcription by RNA polymerase II",
  "term_id": "GO:0006357",
  "gene": "UniProtKB:Q9BRP0",
  "gene_name": "Transcription factor Ovo-like 2",
  "gene_symbol": "OVOL2"
}